{
  "gene_name": "Phospholipase A and acyltransferase 1",
  "gene_symbol": "PLAAT1",
  "term_id": "GO:0008970",
  "term_label": "phospholipase A1 activity",
  "gene": "UniProtKB:Q9HDD0"
}